RIP homotypic interaction motif binding [GO:0071551] (molecular function) Definition: Binding to a RIP homotypic interaction motif (RHIM) of a protein. The RHIM is a 16-amino-acid motif found in some members, including RIP3, of a family of related kinases. Relationships: is a type of protein domain specific binding [GO:0019904] References: PMID:11734559 Sources: GOC:mah Also known as: RHIM binding